cyclodextrin catabolic process [GO:2000901] (biological process) Definition: The chemical reactions and pathways resulting in the breakdown of a cyclodextrin. Sources: GOC:mengo_curators Also known as: cyclodextrin catabolism Relationships: is a type of oligosaccharide catabolic process [GO:0009313]; is a type of GO:1901027; is a type of cyclodextrin metabolic process [GO:2000900] Regulation: regulated by regulation of cyclodextrin catabolic process [GO:2000957]; negatively regulated by GO:2000958; positively regulated by positive regulation of cyclodextrin catabolic process [GO:2000959]